{
  "gene": "UniProtKB:Q8NGQ6",
  "term_label": "odorant binding",
  "gene_symbol": "OR9I1",
  "gene_name": "Olfactory receptor 9I1",
  "term_id": "GO:0005549"
}